{
  "term_label": "mitochondrial permeability transition pore complex",
  "gene_name": "ADP_ATP translocase 3",
  "gene": "UniProtKB:P12236",
  "gene_symbol": "SLC25A6",
  "term_id": "GO:0005757"
}